regulation of iron ion import across plasma membrane [GO:1904438] (biological process) References: PMID:18353247 Sources: GOC:BHF, GOC:TermGenie, GOC:kom, GO_REF:0000058 Relationships: is a type of regulation of iron ion transmembrane transport [GO:0034759]; is a type of regulation of cellular localization [GO:0060341]; regulates GO:0098711 Definition: Any process that modulates the frequency, rate or extent of iron ions import across plasma membrane. Also known as: regulation of ferrous ion import into cell, regulation of ferrous iron import across plasma membrane, regulation of ferrous iron import into cell Subtypes: negative regulation of iron ion import across plasma membrane [GO:1904439], GO:1904440